fructose 1,6-bisphosphate metabolic process [GO:0030388] (biological process) Regulation: positively regulated by positive regulation of fructose 1,6-bisphosphate metabolic process [GO:0060552] Relationships: is a type of phosphate-containing compound metabolic process [GO:0006796]; is a type of organophosphate metabolic process [GO:0019637]; is a type of carbohydrate derivative metabolic process [GO:1901135] Sources: ISBN:0198506732 Definition: The chemical reactions and pathways involving fructose 1,6-bisphosphate, also known as FBP. The D enantiomer is a metabolic intermediate in glycolysis and gluconeogenesis. Also known as: fructose 1,6-bisphosphate metabolism